{
  "gene_name": "Keratin-associated protein 2-3",
  "term_label": "Unknown cellular component",
  "gene": "UniProtKB:P0C7H8",
  "term_id": "UNKNOWN:0003",
  "gene_symbol": "KRTAP2-3"
}